{
  "term_label": "cytoplasmic stress granule",
  "gene_name": "Rho-associated protein kinase 1",
  "gene": "UniProtKB:Q13464",
  "gene_symbol": "ROCK1",
  "term_id": "GO:0010494"
}